central cylinder [GO:1990805] (cellular component) Definition: A scaffolding structure present within the inner region of the ciliary transition zone. The central cylinder lies between the outer doublet and inner singlet microtubules. Relationships: is a type of GO:0110165; BFO_0000050 ciliary transition zone [GO:0035869] References: PMID:2428682, PMID:26124290 Sources: GOC:kmv